{
  "term_id": "GO:0000978",
  "term_label": "RNA polymerase II cis-regulatory region sequence-specific DNA binding",
  "gene": "UniProtKB:Q03060",
  "gene_name": "cAMP-responsive element modulator",
  "gene_symbol": "CREM"
}